{
  "gene": "UniProtKB:P02708",
  "term_id": "GO:0045202",
  "gene_name": "Acetylcholine receptor subunit alpha",
  "term_label": "synapse",
  "gene_symbol": "CHRNA1"
}